{
  "term_id": "GO:0008467",
  "gene": "UniProtKB:Q9Y662",
  "term_label": "[heparan sulfate]-glucosamine 3-sulfotransferase activity",
  "gene_name": "Heparan sulfate glucosamine 3-O-sulfotransferase 3B1",
  "gene_symbol": "HS3ST3B1"
}